{
  "gene_name": "Uncharacterized protein C19orf47",
  "gene_symbol": "C19orf47",
  "gene": "UniProtKB:Q8N9M1",
  "term_id": "UNKNOWN:0002",
  "term_label": "Unknown biological process"
}